{
  "gene_symbol": "SPATS2",
  "term_label": "cytoplasm",
  "gene_name": "Spermatogenesis-associated serine-rich protein 2",
  "term_id": "GO:0005737",
  "gene": "UniProtKB:Q86XZ4"
}